{
  "gene_symbol": "THBS4",
  "gene_name": "Thrombospondin-4",
  "term_id": "GO:0034976",
  "term_label": "response to endoplasmic reticulum stress",
  "gene": "UniProtKB:P35443"
}